{
  "term_id": "GO:0045576",
  "term_label": "mast cell activation",
  "gene": "UniProtKB:Q13094",
  "gene_name": "Lymphocyte cytosolic protein 2",
  "gene_symbol": "LCP2"
}